{
  "gene_symbol": "CIZ1",
  "gene": "UniProtKB:Q9ULV3",
  "term_id": "UNKNOWN:0002",
  "gene_name": "Cip1-interacting zinc finger protein",
  "term_label": "Unknown biological process"
}